{
  "gene": "UniProtKB:Q9NRI7",
  "gene_symbol": "PPY2P",
  "term_id": "UNKNOWN:0001",
  "term_label": "Unknown molecular function",
  "gene_name": "Putative pancreatic polypeptide 2"
}